{
  "gene": "UniProtKB:Q8TC27",
  "gene_symbol": "ADAM32",
  "term_label": "male gonad development",
  "term_id": "GO:0008584",
  "gene_name": "Disintegrin and metalloproteinase domain-containing protein 32"
}